{
  "term_id": "GO:0007218",
  "gene_symbol": "NMUR1",
  "gene_name": "Neuromedin-U receptor 1",
  "term_label": "neuropeptide signaling pathway",
  "gene": "UniProtKB:Q9HB89"
}